{
  "gene_symbol": "MOB3B",
  "gene": "UniProtKB:Q86TA1",
  "gene_name": "MOB kinase activator 3B",
  "term_id": "GO:0005634",
  "term_label": "nucleus"
}